{
  "term_label": "Unknown molecular function",
  "term_id": "UNKNOWN:0001",
  "gene_symbol": "A0A7I2V4U8",
  "gene_name": "Uncharacterized protein",
  "gene": "UniProtKB:A0A7I2V4U8"
}